transmembrane monodehydroascorbate reductase activity [GO:0140575] (molecular function) Definition: Oxidation of monodehydroascorbate outside of a membrane coupled to the reduction of L-ascorbate to monodehydro-L-ascorbate radical on the inner side of a membrane. Electrons get transferred across the membrane during the reaction. References: PMID:1623014 Sources: RHEA:66524 Relationships: is a type of oxidoreductase activity [GO:0016491]